{
  "term_id": "GO:0005764",
  "gene": "UniProtKB:Q9NQE7",
  "gene_symbol": "PRSS16",
  "term_label": "lysosome",
  "gene_name": "Thymus-specific serine protease"
}